{
  "gene": "UniProtKB:Q9UGJ1",
  "term_label": "spindle assembly",
  "gene_name": "Gamma-tubulin complex component 4",
  "term_id": "GO:0051225",
  "gene_symbol": "TUBGCP4"
}